{
  "term_id": "GO:0038110",
  "gene_symbol": "IL2RB",
  "gene_name": "Interleukin-2 receptor subunit beta",
  "gene": "UniProtKB:P14784",
  "term_label": "interleukin-2-mediated signaling pathway"
}